{
  "term_id": "GO:0031012",
  "term_label": "extracellular matrix",
  "gene": "UniProtKB:O75443",
  "gene_symbol": "TECTA",
  "gene_name": "Alpha-tectorin"
}